{
  "term_id": "GO:0090090",
  "gene_name": "Transducin-like enhancer protein 1",
  "gene": "UniProtKB:Q04724",
  "gene_symbol": "TLE1",
  "term_label": "negative regulation of canonical Wnt signaling pathway"
}